{
  "gene_name": "Tumor necrosis factor receptor superfamily member 13B",
  "term_id": "GO:0001782",
  "gene": "UniProtKB:O14836",
  "gene_symbol": "TNFRSF13B",
  "term_label": "B cell homeostasis"
}